{
  "term_label": "Unknown cellular component",
  "gene_symbol": "RPL22",
  "gene_name": "Large ribosomal subunit protein eL22",
  "gene": "UniProtKB:P35268",
  "term_id": "UNKNOWN:0003"
}